{
  "gene": "UniProtKB:Q8TEW6",
  "gene_symbol": "DOK4",
  "term_label": "mitochondrion",
  "gene_name": "Docking protein 4",
  "term_id": "GO:0005739"
}